{
  "term_id": "GO:0005634",
  "gene_symbol": "XRN2",
  "gene": "UniProtKB:Q9H0D6",
  "gene_name": "5'-3' exoribonuclease 2",
  "term_label": "nucleus"
}